{
  "gene_symbol": "KRTAP5-10",
  "gene": "UniProtKB:Q6L8G5",
  "gene_name": "Keratin-associated protein 5-10",
  "term_label": "Unknown cellular component",
  "term_id": "UNKNOWN:0003"
}